{
  "term_label": "plasma membrane",
  "gene_symbol": "ALPP",
  "term_id": "GO:0005886",
  "gene_name": "Alkaline phosphatase, placental type",
  "gene": "UniProtKB:P05187"
}